{
  "gene": "UniProtKB:Q8NEG7",
  "term_id": "GO:0005085",
  "gene_name": "Protein DENND6B",
  "gene_symbol": "DENND6B",
  "term_label": "guanyl-nucleotide exchange factor activity"
}